{
  "gene_symbol": "DNAJC17",
  "gene": "UniProtKB:Q9NVM6",
  "gene_name": "DnaJ homolog subfamily C member 17",
  "term_label": "Unknown molecular function",
  "term_id": "UNKNOWN:0001"
}